{
  "gene_name": "Microtubule-associated proteins 1A_1B light chain 3 beta 2",
  "gene": "UniProtKB:A6NCE7",
  "gene_symbol": "MAP1LC3B2",
  "term_label": "mitophagy",
  "term_id": "GO:0000423"
}